{
  "gene_name": "Eukaryotic translation initiation factor 3 subunit F",
  "term_label": "eukaryotic translation initiation factor 3 complex, eIF3m",
  "gene": "UniProtKB:O00303",
  "gene_symbol": "EIF3F",
  "term_id": "GO:0071541"
}